{
  "gene_symbol": "HOXA10",
  "gene": "UniProtKB:P31260",
  "gene_name": "Homeobox protein Hox-A10",
  "term_label": "DNA-binding transcription factor activity, RNA polymerase II-specific",
  "term_id": "GO:0000981"
}